{
  "gene_symbol": "MOGAT1",
  "term_id": "GO:0019432",
  "gene": "UniProtKB:Q96PD6",
  "gene_name": "2-acylglycerol O-acyltransferase 1",
  "term_label": "triglyceride biosynthetic process"
}